fungal-type vacuole [GO:0000324] (cellular component) Also known as: vacuole, cell cycle-correlated morphology Relationships: is a type of storage vacuole [GO:0000322]; is a type of lytic vacuole [GO:0000323] Definition: A vacuole that has both lytic and storage functions. The fungal vacuole is a large, membrane-bounded organelle that functions as a reservoir for the storage of small molecules (including polyphosphate, amino acids, several divalent cations (e.g. calcium), other ions, and other small molecules) as well as being the primary compartment for degradation. It is an acidic compartment, containing an ensemble of acid hydrolases. At least in S. cerevisiae, there are indications that the morphology of the vacuole is variable and correlated with the cell cycle, with logarithmically growing cells having a multilobed, reticulated vacuole, while stationary phase cells contain a single large structure. Sources: GOC:mah, GOC:mtg_sensu, ISBN:0879693649